manganese ion binding [GO:0030145] (molecular function) Definition: Binding to a manganese ion (Mn). Sources: GOC:ai Relationships: is a type of transition metal ion binding [GO:0046914] Also known as: Mn binding, manganese binding